{
  "term_label": "ATP hydrolysis activity",
  "gene_name": "ATP-dependent Clp protease ATP-binding subunit clpX-like, mitochondrial",
  "term_id": "GO:0016887",
  "gene": "UniProtKB:O76031",
  "gene_symbol": "CLPX"
}